{
  "term_id": "UNKNOWN:0001",
  "gene_name": "Phosducin-like protein",
  "gene_symbol": "PDCL",
  "gene": "UniProtKB:Q13371",
  "term_label": "Unknown molecular function"
}